{
  "gene_symbol": "ACLY",
  "term_label": "fatty acid biosynthetic process",
  "gene": "UniProtKB:P53396",
  "term_id": "GO:0006633",
  "gene_name": "ATP-citrate synthase"
}